{
  "term_id": "GO:0005243",
  "gene_name": "Gap junction beta-5 protein",
  "gene_symbol": "GJB5",
  "gene": "UniProtKB:O95377",
  "term_label": "gap junction channel activity"
}